response to chitin [GO:0010200] (biological process) Relationships: is a type of response to nitrogen compound [GO:1901698]; is a type of GO:1901700 Sources: GOC:sm Definition: A process that results in a change in state or activity of a cell or an organism (in terms of movement, secretion, enzyme production, gene expression, etc.) as a result of a chitin stimulus. Subtypes: cellular response to chitin [GO:0071323]